{
  "gene_symbol": "YWHAH",
  "gene": "UniProtKB:Q04917",
  "gene_name": "14-3-3 protein eta",
  "term_label": "Unknown molecular function",
  "term_id": "UNKNOWN:0001"
}